{
  "term_label": "DNA-binding transcription factor activity, RNA polymerase II-specific",
  "term_id": "GO:0000981",
  "gene_symbol": "SHOX2",
  "gene_name": "Short stature homeobox protein 2",
  "gene": "UniProtKB:O60902"
}